{
  "gene": "UniProtKB:Q9H3J6",
  "gene_symbol": "MTRFR",
  "term_label": "mitochondrion",
  "term_id": "GO:0005739",
  "gene_name": "Mitochondrial translation release factor in rescue"
}